dolichyl-diphosphooligosaccharide-protein glycotransferase activity [GO:0004579] (molecular function) Definition: Catalysis of the reaction: dolichyl diphosphooligosaccharide + protein L-asparagine = dolichyl diphosphate + a glycoprotein with the oligosaccharide chain attached by glycosylamine linkage to protein L-asparagine. Sources: RHEA:22980 Also known as: asparagine N-glycosyltransferase activity, dolichyl-diphosphooligosaccharide-protein glycosyltransferase activity, dolichyl-diphosphooligosaccharide:protein-L-asparagine oligopolysaccharidotransferase activity, dolichyldiphosphooligosaccharide-protein glycosyltransferase activity, dolichyldiphosphooligosaccharide-protein oligosaccharyltransferase activity, dolichyldiphosphoryloligosaccharide-protein oligosaccharyltransferase activity, dolichylpyrophosphodiacetylchitobiose-protein glycosyltransferase activity, oligomannosyltransferase activity Relationships: is a type of oligosaccharyl transferase activity [GO:0004576]